esBAF complex [GO:0140093] (cellular component) Also known as: embryonic stem cell-specific BAF complex, embryonic stem cell-specific SWI/SNF complex Relationships: is a type of SWI/SNF superfamily-type complex [GO:0070603] Definition: An embryonic stem cell-specific SWI/SNF-type complex that contains eight or nine proteins, including both conserved (core) and nonconserved components; contains the ATPase product of either the SMARCA4/BAF190A/BRG1 gene, the mammalian ortholog of the yeast SNF2 gene, or an ortholog thereof. Compared to many other BAF complexes never contains ACTL6B/BAF53B, ARID1B/BAF250B, SMARCA2/BRM, SMARCC2/BAF170 or SMARCD3/BAF60C but contains PHF10/BAF45A, DPF2/BAF45D and possibly one of BCL7A/B/C. References: PMID:19279218, PMID:19279220, PMID:2620226, PMID:8804307, PMID:8895581 Sources: GOC:bhm